{
  "term_label": "fatty acid biosynthetic process",
  "gene_symbol": "PNLIPRP2",
  "term_id": "GO:0006633",
  "gene_name": "Pancreatic lipase-related protein 2",
  "gene": "UniProtKB:P54317"
}